{
  "gene_symbol": "YIPF1",
  "term_label": "Golgi apparatus",
  "term_id": "GO:0005794",
  "gene_name": "Protein YIPF1",
  "gene": "UniProtKB:Q9Y548"
}